{
  "gene_symbol": "PICALM",
  "gene": "UniProtKB:Q13492",
  "term_id": "GO:0032050",
  "gene_name": "Phosphatidylinositol-binding clathrin assembly protein",
  "term_label": "clathrin heavy chain binding"
}